{
  "term_id": "GO:0045202",
  "gene_symbol": "GPC6",
  "term_label": "synapse",
  "gene_name": "Glypican-6",
  "gene": "UniProtKB:Q9Y625"
}